glutarate-semialdehyde dehydrogenase (NADP+) activity [GO:0102810] (molecular function) Sources: GOC:pz, RHEA:57832 Relationships: is a type of GO:0016620 Definition: Catalysis of the reaction: 5-oxopentanoate + NADP + H2O = glutarate + NADPH + 2 H+.